negative regulation of dopamine uptake involved in synaptic transmission [GO:0051585] (biological process) Subtypes: inhibition of dopamine uptake involved in synaptic transmission [GO:0051587] Also known as: down regulation of dopamine uptake involved in synaptic transmission, down-regulation of dopamine uptake involved in synaptic transmission, downregulation of dopamine uptake involved in synaptic transmission, negative regulation of dopamine import involved in synaptic transmission Sources: GOC:ai Relationships: is a type of regulation of dopamine uptake involved in synaptic transmission [GO:0051584]; is a type of GO:0051945; negatively regulates GO:0051583 Definition: Any process that stops, prevents, or reduces the frequency, rate or extent of the directed movement of dopamine into a presynaptic neuron or glial cell.